glucan 1,3-alpha-glucosidase activity [GO:0033919] (molecular function) Definition: Catalysis of the hydrolysis of terminal (1->3)-alpha-D-glucosidic links in 1,3-alpha-D-glucans. Relationships: is a type of alpha-glucosidase activity [GO:0090599] Sources: EC:3.2.1.84 Also known as: 1,3-alpha-D-glucan 3-glucohydrolase activity, exo-1,3-alpha-glucanase activity